{
  "gene": "UniProtKB:O00634",
  "term_label": "Unknown cellular component",
  "gene_symbol": "NTN3",
  "gene_name": "Netrin-3",
  "term_id": "UNKNOWN:0003"
}